{
  "term_label": "antigen binding",
  "gene_name": "Ficolin-3",
  "gene_symbol": "FCN3",
  "term_id": "GO:0003823",
  "gene": "UniProtKB:O75636"
}